{
  "gene_name": "GRB10-interacting GYF protein 2",
  "term_id": "GO:0016020",
  "gene": "UniProtKB:Q6Y7W6",
  "term_label": "membrane",
  "gene_symbol": "GIGYF2"
}